{
  "gene_symbol": "ABCA1",
  "term_id": "UNKNOWN:0003",
  "gene_name": "Phospholipid-transporting ATPase ABCA1",
  "term_label": "Unknown cellular component",
  "gene": "UniProtKB:O95477"
}